{
  "gene_name": "Sialidase-2",
  "term_label": "oligosaccharide catabolic process",
  "term_id": "GO:0009313",
  "gene_symbol": "NEU2",
  "gene": "UniProtKB:Q9Y3R4"
}